p-coumarate 3-hydroxylase activity [GO:0046409] (MF) References: PMID:11429408, PMID:11891223 Relationships: is a type of monooxygenase activity [GO:0004497] Definition: Catalysis of the reaction: shikimate or quinate ester of p-coumaric acid + NADPH + H+ + O2 = caffeic acid conjugate (caffeoyl shikimic acid or chlorogenic acid) + H2O + NADP+. Also known as: cytochrome P450 CYP98A3